negative regulation of anterior head development [GO:2000743] (biological process) Relationships: is a type of negative regulation of developmental process [GO:0051093]; is a type of regulation of anterior head development [GO:2000742]; negatively regulates anterior head development [GO:0097065] Sources: GOC:obol Definition: Any process that stops, prevents or reduces the frequency, rate or extent of anterior head development.